{
  "term_label": "lactate:proton symporter activity",
  "gene_name": "Monocarboxylate transporter 4",
  "gene_symbol": "SLC16A3",
  "gene": "UniProtKB:O15427",
  "term_id": "GO:0015650"
}